{
  "term_id": "GO:0006357",
  "term_label": "regulation of transcription by RNA polymerase II",
  "gene_symbol": "ZBTB42",
  "gene": "UniProtKB:B2RXF5",
  "gene_name": "Zinc finger and BTB domain-containing protein 42"
}